{
  "gene": "UniProtKB:P08833",
  "gene_name": "Insulin-like growth factor-binding protein 1",
  "term_id": "GO:0031995",
  "term_label": "insulin-like growth factor II binding",
  "gene_symbol": "IGFBP1"
}